{
  "term_label": "humoral immune response",
  "gene_symbol": "TNFRSF21",
  "term_id": "GO:0006959",
  "gene_name": "Tumor necrosis factor receptor superfamily member 21",
  "gene": "UniProtKB:O75509"
}